riboflavin synthase activity [GO:0004746] (molecular function) Relationships: is a type of GO:0016765 Sources: EC:2.5.1.9, RHEA:20772 Definition: Catalysis of the reaction: 2 6,7-dimethyl-8-(1-D-ribityl)lumazine + H+ = 5-amino-6-(D-ribitylamino)uracil + riboflavin. Also known as: vitamin B2 synthase activity, heavy riboflavin synthase, light riboflavin synthase, 6,7-dimethyl-8-(1-D-ribityl)lumazine:6,7-dimethyl-8-(1-D-ribityl)lumazine 2,3-butanediyltransferase activity, riboflavin synthetase activity, riboflavine synthase activity, riboflavine synthetase activity